{
  "gene": "UniProtKB:O95222",
  "gene_symbol": "OR6A2",
  "gene_name": "Olfactory receptor 6A2",
  "term_label": "detection of chemical stimulus involved in sensory perception of smell",
  "term_id": "GO:0050911"
}